{
  "gene_name": "Putative spermatogenesis-associated protein 31C1",
  "gene_symbol": "SPATA31C1",
  "term_label": "Unknown cellular component",
  "gene": "UniProtKB:P0DKV0",
  "term_id": "UNKNOWN:0003"
}